negative regulation of myoblast fusion [GO:1901740] (biological process) Definition: Any process that stops, prevents or reduces the frequency, rate or extent of myoblast fusion. Relationships: is a type of negative regulation of syncytium formation by plasma membrane fusion [GO:0034242]; is a type of regulation of myoblast fusion [GO:1901739]; negatively regulates myoblast fusion [GO:0007520] References: PMID:21364645 Sources: GOC:BHF, GOC:TermGenie, GOC:rl Also known as: down regulation of myoblast fusion, down-regulation of myoblast fusion, downregulation of myoblast fusion, inhibition of myoblast fusion